axonal defasciculation [GO:0007414] (biological process) Also known as: defasciculation of neuron Definition: Separation of axons away from a bundle of axons known as a fascicle. Subtypes: defasciculation of motor neuron axon [GO:0007415] Relationships: is a type of neuron recognition [GO:0008038]; is part of GO:0061564 Sources: GOC:dgh, ISBN:039751820X